N-glutamylanilide hydrolase activity [GO:0102572] (molecular function) Sources: GOC:pz Relationships: is_a hydrolase activity, acting on carbon-nitrogen (but not peptide) bonds, in linear amides [GO:0016811] Definition: Catalysis of the reaction: N5-phenyl-L-glutamine + H2O = L-glutamate + aniline + H+.